negative regulation of histamine secretion by mast cell [GO:1903594] (biological process) Relationships: is a type of negative regulation of hormone secretion [GO:0046888]; is a type of negative regulation of inflammatory response [GO:0050728]; is a type of regulation of histamine secretion by mast cell [GO:1903593]; negatively regulates histamine secretion by mast cell [GO:0002553] Definition: Any process that stops, prevents or reduces the frequency, rate or extent of histamine secretion by mast cell. References: PMID:18253931 Sources: GOC:TermGenie, GOC:als, GO_REF:0000058 Also known as: down regulation of histamine secretion by mast cell, down-regulation of histamine secretion by mast cell, downregulation of histamine secretion by mast cell, inhibition of histamine secretion by mast cell